{
  "gene_symbol": "TFAM",
  "gene_name": "Transcription factor A, mitochondrial",
  "term_label": "mitochondrial transcription factor activity",
  "gene": "UniProtKB:Q00059",
  "term_id": "GO:0034246"
}